{
  "gene": "UniProtKB:O15146",
  "gene_symbol": "MUSK",
  "term_label": "transmembrane receptor protein tyrosine kinase activity",
  "term_id": "GO:0004714",
  "gene_name": "Muscle, skeletal receptor tyrosine-protein kinase"
}